{
  "term_id": "GO:0000978",
  "gene_name": "Dachshund homolog 2",
  "gene_symbol": "DACH2",
  "gene": "UniProtKB:Q96NX9",
  "term_label": "RNA polymerase II cis-regulatory region sequence-specific DNA binding"
}